{
  "gene": "UniProtKB:Q9NQC7",
  "term_label": "protein K63-linked deubiquitination",
  "gene_name": "Ubiquitin carboxyl-terminal hydrolase CYLD",
  "term_id": "GO:0070536",
  "gene_symbol": "CYLD"
}